{
  "term_id": "GO:0086002",
  "term_label": "cardiac muscle cell action potential involved in contraction",
  "gene_symbol": "SCN1B",
  "gene_name": "Sodium channel subunit beta-1",
  "gene": "UniProtKB:Q07699"
}